{
  "gene_name": "Sorting nexin-24",
  "gene": "UniProtKB:Q9Y343",
  "gene_symbol": "SNX24",
  "term_label": "Unknown cellular component",
  "term_id": "UNKNOWN:0003"
}